{
  "gene": "UniProtKB:P25205",
  "gene_symbol": "MCM3",
  "gene_name": "DNA replication licensing factor MCM3",
  "term_id": "GO:0003697",
  "term_label": "single-stranded DNA binding"
}